{
  "term_label": "cellular response to copper ion",
  "gene_symbol": "MT1G",
  "gene": "UniProtKB:P13640",
  "gene_name": "Metallothionein-1G",
  "term_id": "GO:0071280"
}